negative regulation of blood-brain barrier permeability [GO:1905604] (biological process) Definition: Any process that decreases blood-brain barrier permeability, the quality of the blood-brain barrier that allows for a controlled passage of substances (e.g. macromolecules, small molecules, ions) into and out of the brain. Relationships: is a type of GO:0043116; is a type of GO:1905603 References: PMID:22524708, PMID:30280653 Sources: GOC:TermGenie, GOC:als, GOC:aruk, GOC:bc, GO_REF:0000058 Also known as: down-regulation of BBB permeability, down-regulation of blood-brain barrier permeability, down-regulation of blood/brain barrier permeability, downregulation of BBB permeability, downregulation of blood-brain barrier permeability, downregulation of blood/brain barrier permeability, negative regulation of BBB permeability, negative regulation of blood/brain barrier permeability, inhibition of maintenance of permeability of BBB, inhibition of maintenance of permeability of blood-brain barrier